{
  "gene": "UniProtKB:P14136",
  "term_label": "intermediate filament organization",
  "gene_name": "Glial fibrillary acidic protein",
  "term_id": "GO:0045109",
  "gene_symbol": "GFAP"
}